{
  "gene": "UniProtKB:Q96T83",
  "term_label": "regulation of intracellular pH",
  "gene_name": "Sodium_hydrogen exchanger 7",
  "gene_symbol": "SLC9A7",
  "term_id": "GO:0051453"
}